RNA 2'-O-methyltransferase activity [GO:0062105] (molecular function) Relationships: is a type of O-methyltransferase activity [GO:0008171]; is a type of RNA methyltransferase activity [GO:0008173] References: PMID:30626973 Sources: RHEA:58956 Definition: Catalysis of the reaction: S-adenosyl-L-methionine + RNA = S-adenosyl-L-homocysteine + RNA containing 2'-O-methylribonucleotide. Subtypes: GO:0008650, 23S rRNA (adenosine(1067)-2'-O)-methyltransferase activity [GO:0030743], rRNA (guanosine-2'-O-)-methyltransferase activity [GO:0070039], rRNA (cytosine-2'-O-)-methyltransferase activity [GO:0070677], GO:0090486, tRNA 2'-O-methyltransferase activity [GO:0106050]